protein complex involved in cell-cell adhesion [GO:0098635] (cellular component) Sources: GOC:dos Relationships: is a type of GO:0098636 Subtypes: galectin lattice [GO:0140366], galectin complex [GO:1990724] Definition: Any protein complex that is capable of carrying out some part of the process of cell-cell adhesion.